{
  "gene_symbol": "R3HCC1",
  "gene_name": "R3H and coiled-coil domain-containing protein 1",
  "term_id": "UNKNOWN:0003",
  "gene": "UniProtKB:Q9Y3T6",
  "term_label": "Unknown cellular component"
}